{
  "gene_name": "Neuromedin-S",
  "term_id": "UNKNOWN:0001",
  "gene_symbol": "NMS",
  "gene": "UniProtKB:Q5H8A3",
  "term_label": "Unknown molecular function"
}